{
  "term_label": "transcription initiation at RNA polymerase II promoter",
  "term_id": "GO:0006367",
  "gene_symbol": "TAF5",
  "gene_name": "Transcription initiation factor TFIID subunit 5",
  "gene": "UniProtKB:Q15542"
}